{
  "gene": "UniProtKB:P10827",
  "gene_symbol": "THRA",
  "term_id": "GO:0048384",
  "gene_name": "Thyroid hormone receptor alpha",
  "term_label": "retinoic acid receptor signaling pathway"
}